{
  "gene_symbol": "ACO1",
  "gene": "UniProtKB:P21399",
  "gene_name": "Cytoplasmic aconitate hydratase",
  "term_label": "cytosol",
  "term_id": "GO:0005829"
}